{
  "gene": "UniProtKB:Q14657",
  "gene_name": "EKC_KEOPS complex subunit LAGE3",
  "term_id": "GO:0070525",
  "term_label": "tRNA threonylcarbamoyladenosine metabolic process",
  "gene_symbol": "LAGE3"
}